exogen [GO:0042638] (biological process) Relationships: is a type of hair cycle phase [GO:0044851]; is part of hair follicle maturation [GO:0048820] Regulation: RO_0002211 by regulation of timing of exogen [GO:0051887]; positively regulated by positive regulation of timing of exogen [GO:0051888]; negatively regulated by GO:0051889 Definition: The shedding phase of the hair cycle. Also known as: hair shedding Note: Note that this term should not be used for direct annotation. If you are trying to make an annotation to x phase, it is likely that the correct annotation is 'regulation of x/y phase transition' or to a process which occurs during the reported phase. To capture the phase when a specific location or process is observed, the phase term can be used in an annotation extension (PMID:24885854) applied to a cellular component term (with the relation exists_during) or a biological process term (with the relation happens_during). References: PMID:12230507